{
  "gene_symbol": "CDH10",
  "gene_name": "Cadherin-10",
  "term_id": "GO:0007043",
  "gene": "UniProtKB:Q9Y6N8",
  "term_label": "cell-cell junction assembly"
}